{
  "gene_symbol": "FAM234B",
  "term_label": "Unknown molecular function",
  "gene": "UniProtKB:A2RU67",
  "gene_name": "Protein FAM234B",
  "term_id": "UNKNOWN:0001"
}